{
  "term_label": "positive regulation of cilium assembly",
  "gene_symbol": "TAPT1",
  "gene": "UniProtKB:Q6NXT6",
  "gene_name": "Transmembrane anterior posterior transformation protein 1 homolog",
  "term_id": "GO:0045724"
}